{
  "term_label": "Unknown molecular function",
  "gene_name": "Transforming acidic coiled-coil-containing protein 3",
  "gene_symbol": "TACC3",
  "gene": "UniProtKB:Q9Y6A5",
  "term_id": "UNKNOWN:0001"
}